positive regulation of iron export across plasma membrane [GO:1904040] (biological process) Also known as: activation of ferrous iron export, activation of iron(2+) export, positive regulation of ferrous iron export, positive regulation of iron(2+) export, up regulation of ferrous iron export, up regulation of iron(2+) export, up-regulation of ferrous iron export, up-regulation of iron(2+) export, upregulation of ferrous iron export, upregulation of iron(2+) export References: PMID:15514116 Sources: GOC:BHF, GOC:TermGenie, GOC:kom, GO_REF:0000058 Definition: Any process that activates or increases the frequency, rate or extent of export of iron ions from inside of a cell, across the plasma membrane and into the extracellular region. Relationships: is a type of positive regulation of iron ion transmembrane transport [GO:0034761]; is a type of GO:1904038; positively regulates iron ion export across plasma membrane [GO:1903988]